{
  "gene_symbol": "TNFRSF12A",
  "gene": "UniProtKB:Q9NP84",
  "term_label": "positive regulation of extrinsic apoptotic signaling pathway",
  "gene_name": "Tumor necrosis factor receptor superfamily member 12A",
  "term_id": "GO:2001238"
}